{
  "term_label": "cytoplasm",
  "gene_symbol": "MYO7B",
  "gene_name": "Unconventional myosin-VIIb",
  "term_id": "GO:0005737",
  "gene": "UniProtKB:Q6PIF6"
}